{
  "gene": "UniProtKB:P49441",
  "gene_symbol": "INPP1",
  "term_label": "inositol-1,4-bisphosphate 1-phosphatase activity",
  "gene_name": "Inositol polyphosphate 1-phosphatase",
  "term_id": "GO:0004441"
}